{
  "term_label": "Unknown biological process",
  "gene_name": "Ankyrin repeat domain-containing protein 35",
  "gene": "UniProtKB:Q8N283",
  "gene_symbol": "ANKRD35",
  "term_id": "UNKNOWN:0002"
}